{
  "gene_name": "Small ribosomal subunit protein eS4, X isoform",
  "gene": "UniProtKB:P62701",
  "term_id": "GO:0003723",
  "term_label": "RNA binding",
  "gene_symbol": "RPS4X"
}